ergosteryl 3-beta-D-glucoside catabolic process [GO:1904462] (biological process) Relationships: is a type of steroid catabolic process [GO:0006706]; is a type of saponin catabolic process [GO:0016136]; is a type of beta-glucoside catabolic process [GO:1901805] Definition: The chemical reactions and pathways resulting in the breakdown of ergosteryl 3-beta-D-glucoside. Also known as: ergosteryl 3-beta-D-glucoside breakdown, ergosteryl 3-beta-D-glucoside catabolism, ergosteryl 3-beta-D-glucoside degradation References: PMID:26116408 Sources: GOC:TermGenie, GO_REF:0000068